pericardial nephrocyte differentiation [GO:0061320] (biological process) Also known as: pericardial cell differentiation Definition: The process in which a relatively unspecialized cell acquires the specialized structural and/or functional features of a pericardial nephrocyte. A pericardial nephrocyte is an insect renal cell that filters hemolymph and is found with other pericardial nephrocytes in two rows flanking the dorsal vessel. Differentiation includes the processes involved in commitment of a cell to a specific fate and its subsequent development to the mature state. Relationships: is a type of GO:0061319 References: PMID:19783135 Sources: CL:0000474, GOC:dph, GOC:mtg_kidney_jan10, GOC:sart